{
  "gene_symbol": "ADGRA2",
  "term_label": "Wnt signalosome",
  "gene": "UniProtKB:Q96PE1",
  "term_id": "GO:1990909",
  "gene_name": "Adhesion G protein-coupled receptor A2"
}